{
  "gene_symbol": "CAPNS1",
  "gene": "UniProtKB:P04632",
  "term_id": "UNKNOWN:0001",
  "term_label": "Unknown molecular function",
  "gene_name": "Calpain small subunit 1"
}